{
  "gene_symbol": "KRTAP4-5",
  "gene": "UniProtKB:Q9BYR2",
  "term_label": "Unknown cellular component",
  "gene_name": "Keratin-associated protein 4-5",
  "term_id": "UNKNOWN:0003"
}